{
  "gene_name": "MOB kinase activator 3A",
  "term_label": "nucleus",
  "term_id": "GO:0005634",
  "gene_symbol": "MOB3A",
  "gene": "UniProtKB:Q96BX8"
}